{
  "term_id": "GO:0006289",
  "gene_name": "DNA repair protein complementing XP-C cells",
  "gene_symbol": "XPC",
  "gene": "UniProtKB:Q01831",
  "term_label": "nucleotide-excision repair"
}